{
  "term_id": "GO:0035556",
  "gene_name": "Serine_threonine-protein kinase haspin",
  "gene": "UniProtKB:Q8TF76",
  "gene_symbol": "HASPIN",
  "term_label": "intracellular signal transduction"
}